11-beta-hydroxysteroid dehydrogenase (NADP+) activity [GO:0070524] (molecular function) Definition: Catalysis of the reaction: an 11-beta-hydroxysteroid + NADP+ = an 11-oxosteroid + NADPH + H+. References: PMID:16216911 Sources: RHEA:11388 Also known as: beta-hydroxysteroid dehydrogenase, corticosteroid 11-beta-dehydrogenase activity Relationships: is a type of steroid dehydrogenase activity, acting on the CH-OH group of donors, NAD or NADP as acceptor [GO:0033764] Subtypes: GO:0102196